{
  "gene_name": "Small ribosomal subunit protein mS35",
  "gene_symbol": "MRPS35",
  "term_label": "Unknown biological process",
  "term_id": "UNKNOWN:0002",
  "gene": "UniProtKB:P82673"
}